{
  "gene": "UniProtKB:Q9BXW6",
  "gene_name": "Oxysterol-binding protein-related protein 1",
  "term_label": "cholesterol binding",
  "gene_symbol": "OSBPL1A",
  "term_id": "GO:0015485"
}